2-hydroxy-3-oxoadipate synthase activity [GO:0050439] (molecular function) Definition: Catalysis of the reaction: 2-oxoglutarate + glyoxylate + H+ = 2-hydroxy-3-oxoadipate + CO2. Sources: EC:2.2.1.5, RHEA:14341 Also known as: 2-hydroxy-3-oxoadipate glyoxylate-lyase (carboxylating) activity, 2-hydroxy-3-oxoadipate synthetase activity, 2-oxoglutarate:glyoxylate succinaldehydetransferase (decarboxylating), alpha-ketoglutaric-glyoxylic carboligase activity, oxoglutarate: glyoxylate carboligase activity, oxoglutarate:glyoxylate carboligase activity Relationships: is a type of GO:0016744